secretory granule [GO:0030141] (CC) Definition: A small subcellular vesicle, surrounded by a membrane, that is formed from the Golgi apparatus and contains a highly concentrated protein destined for secretion. Secretory granules move towards the periphery of the cell and upon stimulation, their membranes fuse with the cell membrane, and their protein load is exteriorized. Processing of the contained protein may take place in secretory granules. Note: Note that the term 'secretory vesicle' is sometimes used in this sense, but can also mean 'transport vesicle ; GO:0030133'. Subtypes: GO:0001669, apicomplexan dense granule [GO:0020026], dense core granule [GO:0031045], platelet alpha granule [GO:0031091], insulin-responsive compartment [GO:0032593], Weibel-Palade body [GO:0033093], GO:0036000, specific granule [GO:0042581], azurophil granule [GO:0042582], chromaffin granule [GO:0042583], zymogen granule [GO:0042588], GO:0042599, GO:0042827, cortical granule [GO:0060473], tertiary granule [GO:0070820], mucin granule [GO:0098594], ficolin-1-rich granule [GO:0101002] Also known as: secretory vesicle Relationships: is a type of secretory vesicle [GO:0099503]; is part of endomembrane system [GO:0012505] Sources: GOC:mah, ISBN:0198506732